{
  "term_label": "Unknown molecular function",
  "gene_name": "Immunoglobulin kappa variable 3-20",
  "gene": "UniProtKB:P01619",
  "term_id": "UNKNOWN:0001",
  "gene_symbol": "IGKV3-20"
}